{
  "gene_symbol": "MN1",
  "gene_name": "Transcriptional activator MN1",
  "term_label": "Unknown cellular component",
  "gene": "UniProtKB:Q10571",
  "term_id": "UNKNOWN:0003"
}